{
  "gene_name": "Adenine phosphoribosyltransferase",
  "gene_symbol": "APRT",
  "term_id": "GO:0003999",
  "gene": "UniProtKB:P07741",
  "term_label": "adenine phosphoribosyltransferase activity"
}